{
  "gene_name": "Speriolin-like protein",
  "term_id": "GO:0007283",
  "gene_symbol": "SPATC1L",
  "term_label": "spermatogenesis",
  "gene": "UniProtKB:Q9H0A9"
}